neuron projection cytoplasm [GO:0120111] (cellular component) Subtypes: GO:0032839, axon cytoplasm [GO:1904115] Definition: All of the contents of a plasma membrane bounded neuron projection, excluding the plasma membrane surrounding the projection. Relationships: is a type of GO:0032838; is part of GO:0043005 Sources: GOC:ha